{
  "term_label": "NADPH oxidase complex",
  "gene_symbol": "NCF4",
  "term_id": "GO:0043020",
  "gene_name": "Neutrophil cytosol factor 4",
  "gene": "UniProtKB:Q15080"
}